{
  "term_id": "GO:0006357",
  "gene": "UniProtKB:Q8NEA6",
  "term_label": "regulation of transcription by RNA polymerase II",
  "gene_name": "Zinc finger protein GLIS3",
  "gene_symbol": "GLIS3"
}